{
  "term_id": "GO:0034440",
  "gene_symbol": "ALOX5",
  "term_label": "lipid oxidation",
  "gene_name": "Polyunsaturated fatty acid 5-lipoxygenase",
  "gene": "UniProtKB:P09917"
}